{
  "gene": "UniProtKB:Q9UP65",
  "term_id": "GO:0005829",
  "gene_symbol": "PLA2G4C",
  "gene_name": "Cytosolic phospholipase A2 gamma",
  "term_label": "cytosol"
}